VCP-NPL4-UFD1 AAA ATPase complex assembly [GO:1904210] (biological process) Definition: The aggregation, arrangement and bonding together of a set of components to form a VCP-NPL4-UFD1 AAA ATPase complex. References: PMID:17000876 Sources: GOC:PARL, GOC:TermGenie, GOC:bf, GO_REF:0000079 Also known as: VCP-NPL4-UFD1 AAA ATPase complex formation, p97-Ufd1-Npl4 complex assembly, p97-Ufd1-Npl4 complex formation, Cdc48p-Npl4p-Ufd1p AAA ATPase complex assembly, Cdc48p-Npl4p-Ufd1p AAA ATPase complex formation Relationships: is a type of protein-containing complex assembly [GO:0065003] Regulation: regulated by regulation of VCP-NPL4-UFD1 AAA ATPase complex assembly [GO:1904239]; negatively regulated by GO:1904240; RO_0002213 by positive regulation of VCP-NPL4-UFD1 AAA ATPase complex assembly [GO:1904241]